regulation of positive chemotaxis [GO:0050926] (biological process) Subtypes: positive regulation of positive chemotaxis [GO:0050927], negative regulation of positive chemotaxis [GO:0050928], regulation of positive chemotaxis to cAMP [GO:0061118] Relationships: is a type of regulation of chemotaxis [GO:0050920]; regulates GO:0050918 Definition: Any process that modulates the frequency, rate or extent of the directed movement of a motile cell or organism towards a higher concentration in a concentration gradient of a specific chemical. Sources: GOC:ai